{
  "gene_symbol": "INPP4A",
  "term_id": "GO:0016316",
  "term_label": "phosphatidylinositol-3,4-bisphosphate 4-phosphatase activity",
  "gene": "UniProtKB:Q96PE3",
  "gene_name": "Inositol polyphosphate-4-phosphatase type I A"
}